{
  "term_id": "UNKNOWN:0002",
  "gene_symbol": "HRES1",
  "gene_name": "Putative HTLV-1-related endogenous sequence",
  "term_label": "Unknown biological process",
  "gene": "UniProtKB:P13985"
}